{
  "term_id": "UNKNOWN:0001",
  "term_label": "Unknown molecular function",
  "gene_name": "SCL-interrupting locus protein",
  "gene": "UniProtKB:Q15468",
  "gene_symbol": "STIL"
}